dAMP phosphorylation [GO:0061565] (BP) Definition: The process of introducing a phosphate group into dAMP, deoxyadenosine monophosphate, to produce dADP. Addition of two phosphate groups produces dATP. Relationships: is a type of nucleoside monophosphate phosphorylation [GO:0046940] References: PMID:23416111 Sources: GOC:dph